{
  "term_label": "RNA polymerase II cis-regulatory region sequence-specific DNA binding",
  "gene_symbol": "ZKSCAN3",
  "term_id": "GO:0000978",
  "gene": "UniProtKB:Q9BRR0",
  "gene_name": "Zinc finger protein with KRAB and SCAN domains 3"
}